{
  "term_label": "prostaglandin F synthase activity",
  "term_id": "GO:0047017",
  "gene_symbol": "PRXL2B",
  "gene_name": "Prostamide_prostaglandin F synthase",
  "gene": "UniProtKB:Q8TBF2"
}